{
  "term_id": "GO:0031462",
  "gene_name": "Cullin-2",
  "gene": "UniProtKB:Q13617",
  "gene_symbol": "CUL2",
  "term_label": "Cul2-RING ubiquitin ligase complex"
}